{
  "gene": "UniProtKB:Q5SQN1",
  "gene_name": "Synaptosomal-associated protein 47",
  "term_label": "SNARE complex",
  "gene_symbol": "SNAP47",
  "term_id": "GO:0031201"
}